queuosine import across plasma membrane [GO:0160287] (biological process) References: PMID:40526720 Relationships: is a type of import across plasma membrane [GO:0098739]; is a type of GO:1901642 Definition: The directed movement of queuosine from outside of a cell, across the plasma membrane and into the cytosol.